{
  "gene_name": "Prolow-density lipoprotein receptor-related protein 1",
  "term_id": "GO:0006898",
  "gene_symbol": "LRP1",
  "gene": "UniProtKB:Q07954",
  "term_label": "receptor-mediated endocytosis"
}